metanephric cap development [GO:0072185] (BP) Sources: GOC:mtg_kidney_jan10 Definition: The biological process whose specific outcome is the progression of the metanephric cap from an initial condition to its mature state. The metanephric cap is formed by the condensation of metanephric mesenchymal cells surrounding the ureteric bud tip. Relationships: is a type of GO:0072075